{
  "gene": "UniProtKB:Q96GX8",
  "term_id": "UNKNOWN:0003",
  "gene_symbol": "C16orf74",
  "gene_name": "Uncharacterized protein C16orf74",
  "term_label": "Unknown cellular component"
}